{
  "term_id": "GO:0000978",
  "gene_symbol": "KCNIP3",
  "gene": "UniProtKB:Q9Y2W7",
  "gene_name": "Calsenilin",
  "term_label": "RNA polymerase II cis-regulatory region sequence-specific DNA binding"
}